{
  "gene": "UniProtKB:Q401N2",
  "term_id": "GO:0034220",
  "gene_symbol": "ZACN",
  "term_label": "monoatomic ion transmembrane transport",
  "gene_name": "Zinc-activated ligand-gated ion channel"
}